{
  "gene_name": "Clarin-1",
  "gene": "UniProtKB:P58418",
  "term_id": "GO:0050957",
  "term_label": "equilibrioception",
  "gene_symbol": "CLRN1"
}